{
  "gene": "UniProtKB:Q5BJE1",
  "gene_symbol": "CCDC178",
  "term_id": "UNKNOWN:0003",
  "gene_name": "Coiled-coil domain-containing protein 178",
  "term_label": "Unknown cellular component"
}